{
  "gene_symbol": "SLC17A8",
  "term_label": "excitatory synapse",
  "term_id": "GO:0060076",
  "gene_name": "Vesicular glutamate transporter 3",
  "gene": "UniProtKB:Q8NDX2"
}